low-density lipoprotein particle disassembly [GO:0090495] (biological process) Definition: The disaggregation of a low-density lipoprotein particle into its constituent components. Sources: GOC:dph, GOC:tb Subtypes: low-density lipoprotein particle disassembly involved in cholesterol transport [GO:0090121] Relationships: is a type of plasma lipoprotein particle disassembly [GO:0071829]